{
  "term_label": "cytoplasm",
  "gene_name": "Guanine nucleotide-binding protein G(q) subunit alpha",
  "term_id": "GO:0005737",
  "gene": "UniProtKB:P50148",
  "gene_symbol": "GNAQ"
}